{
  "term_id": "GO:0047372",
  "gene": "UniProtKB:Q6UXT9",
  "term_label": "monoacylglycerol lipase activity",
  "gene_symbol": "ABHD15",
  "gene_name": "Protein ABHD15"
}